{
  "gene_name": "Golgin subfamily A member 6-like protein 22",
  "term_id": "UNKNOWN:0002",
  "term_label": "Unknown biological process",
  "gene_symbol": "GOLGA6L22",
  "gene": "UniProtKB:H0YM25"
}